{
  "term_label": "regulation of cytokinesis",
  "gene_symbol": "KLHL9",
  "gene": "UniProtKB:Q9P2J3",
  "gene_name": "Kelch-like protein 9",
  "term_id": "GO:0032465"
}